{
  "gene_name": "Septin-14",
  "gene": "UniProtKB:Q6ZU15",
  "gene_symbol": "SEPTIN14",
  "term_label": "septin ring",
  "term_id": "GO:0005940"
}